{
  "term_id": "GO:0051087",
  "term_label": "protein-folding chaperone binding",
  "gene": "UniProtKB:O75953",
  "gene_symbol": "DNAJB5",
  "gene_name": "DnaJ homolog subfamily B member 5"
}